CMP-N-acetylneuraminate transmembrane transporter activity [GO:0005456] (molecular function) Sources: GOC:ai, GOC:mtg_transport, ISBN:0815340729 Also known as: CMP-sialic acid transmembrane transporter activity Relationships: is a type of pyrimidine nucleotide-sugar transmembrane transporter activity [GO:0015165]; is part of CMP-N-acetylneuraminate transmembrane transport [GO:0015782] Definition: Enables the transfer of a CMP-N-acetylneuraminate from one side of a membrane to the other.